{
  "gene": "UniProtKB:P61587",
  "gene_name": "Rho-related GTP-binding protein RhoE",
  "term_label": "GTP binding",
  "term_id": "GO:0005525",
  "gene_symbol": "RND3"
}